ethylbenzene hydroxylase activity [GO:0018693] (molecular function) Sources: EC:1.17.99.2, RHEA:17897 Also known as: ethylbenzene dehydrogenase activity, ethylbenzene:(acceptor) oxidoreductase activity Relationships: is a type of oxidoreductase activity, acting on CH or CH2 groups [GO:0016725] Definition: Catalysis of the reaction: A + ethylbenzene + H2O = (S)-1-phenylethanol + AH(2).